{
  "gene_symbol": "KRT16",
  "gene": "UniProtKB:P08779",
  "term_label": "keratinocyte differentiation",
  "term_id": "GO:0030216",
  "gene_name": "Keratin, type I cytoskeletal 16"
}